{
  "term_id": "GO:0006096",
  "gene": "UniProtKB:P04075",
  "gene_symbol": "ALDOA",
  "term_label": "glycolytic process",
  "gene_name": "Fructose-bisphosphate aldolase A"
}